{
  "gene_name": "Protein ADM2",
  "gene_symbol": "ADM2",
  "term_id": "GO:0005179",
  "gene": "UniProtKB:Q7Z4H4",
  "term_label": "hormone activity"
}